regulation of eosinophil differentiation [GO:0045643] (BP) Subtypes: negative regulation of eosinophil differentiation [GO:0045644], positive regulation of eosinophil differentiation [GO:0045645] Sources: GOC:go_curators Definition: Any process that modulates the frequency, rate or extent of eosinophil differentiation. Relationships: is_a regulation of granulocyte differentiation [GO:0030852]; regulates eosinophil differentiation [GO:0030222]